{
  "term_id": "GO:0005737",
  "gene_name": "Cyclin-dependent kinase 5 activator 2",
  "gene": "UniProtKB:Q13319",
  "gene_symbol": "CDK5R2",
  "term_label": "cytoplasm"
}